antimonite transmembrane transport [GO:0015699] (biological process) Relationships: is a type of GO:0015698; is a type of GO:0055085 Definition: The directed movement of antimonite into, out of or within a cell, or between cells, by means of some agent such as a transporter or pore. Sources: GOC:krc Also known as: antimonite transport